{
  "gene_symbol": "STK17B",
  "gene": "UniProtKB:O94768",
  "term_id": "GO:0035556",
  "term_label": "intracellular signal transduction",
  "gene_name": "Serine_threonine-protein kinase 17B"
}